histone H4K16 deacetylase activity, NAD-dependent [GO:0046970] (molecular function) Definition: Catalysis of the reaction: histone H4 N6-acetyl-L-lysine (position 16) + NAD+ + H2O = histone H4 L-lysine (position 16) + 2''-O-acetyl-ADP-D-ribose + nicotinamide. This reaction transfers an acetyl group attached to a lysine residue in H4K16 to NAD, producing nicotinamide. Also known as: NAD-dependent histone H4-K16 deacetylase activity, NAD-dependent histone H4K16 deacetylase activity, NAD-dependent histone deacetylase activity (H4-K16 specific) References: PMID:28450737 Sources: GOC:vw Relationships: is a type of histone deacetylase activity, NAD-dependent [GO:0017136]; is a type of histone H4K deacetylase activity [GO:0141051] Note: Note that the residue position corresponds to the canonical human H4 histone (UniProtKB:P02309); this residue is conserved across all eukaryotes. Note that the initiation methionine is cleaved, so the first residue is S1.